{
  "gene_symbol": "AKAP9",
  "gene_name": "A-kinase anchor protein 9",
  "gene": "UniProtKB:Q99996",
  "term_label": "microtubule nucleation",
  "term_id": "GO:0007020"
}